generation of mature 3'-end of LSU-rRNA from tricistronic rRNA transcript (SSU-rRNA, 5.8S rRNA, LSU-rRNA) [GO:0000468] (BP) Relationships: is a type of rRNA 3'-end processing [GO:0031125]; is part of maturation of LSU-rRNA from tricistronic rRNA transcript (SSU-rRNA, 5.8S rRNA, LSU-rRNA) [GO:0000463] Definition: Any process involved in generating the mature 3'-end of an LSU-rRNA derived from a tricistronic rRNA transcript that contained the Small SubUnit (SSU) rRNA, the 5.8S rRNA, and the Large SubUnit (LSU) rRNA, in that order, from 5' to 3' along the primary transcript. Also known as: processing at B2 References: PMID:10690410 Sources: GOC:krc